{
  "gene_symbol": "MAP4K1",
  "term_id": "GO:0008349",
  "term_label": "MAP kinase kinase kinase kinase activity",
  "gene": "UniProtKB:Q92918",
  "gene_name": "Mitogen-activated protein kinase kinase kinase kinase 1"
}